{
  "gene": "UniProtKB:Q8NGK5",
  "term_id": "UNKNOWN:0002",
  "term_label": "Unknown biological process",
  "gene_name": "Olfactory receptor 52M1",
  "gene_symbol": "OR52M1"
}